cellular response to isolation stress [GO:0035901] (biological process) References: PMID:20203532 Sources: GOC:bf Also known as: cellular response to social isolation Definition: Any process that results in a change in state or activity of a cell (in terms of movement, secretion, enzyme production, gene expression, etc.) as a result of a lack of contact with other members of the same species. Relationships: is a type of cellular response to stress [GO:0033554]; is a type of response to isolation stress [GO:0035900]